{
  "gene": "UniProtKB:Q9NRG9",
  "gene_name": "Aladin",
  "gene_symbol": "AAAS",
  "term_id": "GO:0006913",
  "term_label": "nucleocytoplasmic transport"
}